{
  "gene": "UniProtKB:P61289",
  "term_id": "GO:0005654",
  "term_label": "nucleoplasm",
  "gene_name": "Proteasome activator complex subunit 3",
  "gene_symbol": "PSME3"
}